regulation of salicylic acid mediated signaling pathway [GO:2000031] (biological process) Relationships: is a type of GO:0009966; regulates salicylic acid mediated signaling pathway [GO:0009863] Subtypes: GO:0080151 Definition: Any process that modulates the frequency, rate or extent of salicylic acid mediated signaling pathway. Sources: GOC:obol Also known as: regulation of salicylic acid mediated signalling pathway